{
  "term_label": "antigen binding",
  "gene": "UniProtKB:A0A0B4J2B8",
  "term_id": "GO:0003823",
  "gene_name": "Immunoglobulin heavy variable 1_OR15-9 (non-functional) (Fragment)",
  "gene_symbol": "IGHV1OR15-9"
}